{
  "term_id": "GO:0005886",
  "gene_name": "Carbonic anhydrase 4",
  "gene_symbol": "CA4",
  "term_label": "plasma membrane",
  "gene": "UniProtKB:P22748"
}